{
  "gene": "UniProtKB:O94964",
  "gene_name": "Protein SOGA1",
  "term_id": "UNKNOWN:0001",
  "gene_symbol": "SOGA1",
  "term_label": "Unknown molecular function"
}